{
  "gene": "UniProtKB:Q96LB9",
  "gene_name": "Peptidoglycan recognition protein 3",
  "gene_symbol": "PGLYRP3",
  "term_label": "defense response to Gram-positive bacterium",
  "term_id": "GO:0050830"
}